{
  "gene": "UniProtKB:Q5JQF8",
  "gene_symbol": "PABPC1L2A",
  "term_id": "GO:0005634",
  "term_label": "nucleus",
  "gene_name": "Polyadenylate-binding protein 1-like 2"
}